deoxyribonuclease IV (phage-T4-induced) activity [GO:0008833] (molecular function) Sources: EC:3.1.21.2 Also known as: DNA-adenine-transferase activity, E. coli endonuclease IV, Escherichia coli endonuclease II, deoxriboendonuclease activity, deoxyribonuclease IV (phage T4-induced) activity, endodeoxyribonuclease IV (phage T(4)-induced) activity, endodeoxyribonuclease IV (phage T4-induced) activity, endonuclease II, endonuclease IV activity, redoxyendonuclease activity Definition: Catalysis of the endonucleolytic cleavage to 5'-phosphooligonucleotide end-products. Relationships: is a type of GO:0016888